regulation of lipid transport [GO:0032368] (biological process) Relationships: is a type of GO:0051049; is a type of GO:1905952; regulates lipid transport [GO:0006869] Subtypes: GO:0007558, negative regulation of lipid transport [GO:0032369], positive regulation of lipid transport [GO:0032370], regulation of sterol transport [GO:0032371], regulation of intracellular lipid transport [GO:0032377], GO:1901506, regulation of lipid transport across blood-brain barrier [GO:1903000], GO:2000191, regulation of steroid hormone secretion [GO:2000831], regulation of androstenedione secretion [GO:2000837], GO:2000840, regulation of testosterone secretion [GO:2000843], regulation of phospholipid transport [GO:2001138] Sources: GOC:mah Definition: Any process that modulates the frequency, rate or extent of the directed movement of lipids into, out of or within a cell, or between cells, by means of some agent such as a transporter or pore.